{
  "term_label": "cell adhesion",
  "gene_symbol": "PCDHB14",
  "gene": "UniProtKB:Q9Y5E9",
  "term_id": "GO:0007155",
  "gene_name": "Protocadherin beta-14"
}